Notch receptor processing [GO:0007220] (BP) Definition: The series of successive proteolytic cleavages of the Notch protein, which result in an active form of the receptor. Also known as: N receptor processing Relationships: is a type of protein metabolic process [GO:0019538] References: PMID:12651094, PMID:14986688